sperm axoneme assembly [GO:0007288] (biological process) Definition: The assembly and organization of the sperm flagellar axoneme, the bundle of microtubules and associated proteins that forms the core of the eukaryotic sperm flagellum, and is responsible for movement. Sources: GOC:bf, GOC:cilia, ISBN:0198547684 Relationships: is a type of developmental process involved in reproduction [GO:0003006]; is a type of GO:0035082; BFO_0000050 sperm flagellum assembly [GO:0120316]